{
  "term_label": "Unknown cellular component",
  "gene_symbol": "NKIRAS2",
  "gene_name": "NF-kappa-B inhibitor-interacting Ras-like protein 2",
  "term_id": "UNKNOWN:0003",
  "gene": "UniProtKB:Q9NYR9"
}